positive regulation of circadian sleep/wake cycle, sleep [GO:0045938] (biological process) Relationships: is a type of positive regulation of circadian rhythm [GO:0042753]; is a type of regulation of circadian sleep/wake cycle, sleep [GO:0045187]; is a type of positive regulation of behavior [GO:0048520]; positively regulates circadian sleep/wake cycle, sleep [GO:0050802] Sources: GOC:go_curators Also known as: positive regulation of sleep, up regulation of circadian sleep/wake cycle, sleep, up-regulation of circadian sleep/wake cycle, sleep, upregulation of circadian sleep/wake cycle, sleep, activation of circadian sleep/wake cycle, sleep, stimulation of circadian sleep/wake cycle, sleep Subtypes: positive regulation of circadian sleep/wake cycle, REM sleep [GO:0046005], positive regulation of circadian sleep/wake cycle, non-REM sleep [GO:0046010] Definition: Any process that activates or increases the duration or quality of sleep, a readily reversible state of reduced awareness and metabolic activity that occurs periodically in many animals.